{
  "term_label": "extracellular space",
  "gene_symbol": "DAND5",
  "gene": "UniProtKB:Q8N907",
  "gene_name": "DAN domain family member 5",
  "term_id": "GO:0005615"
}